{
  "gene_symbol": "MEIS1",
  "term_label": "animal organ morphogenesis",
  "gene_name": "Homeobox protein Meis1",
  "term_id": "GO:0009887",
  "gene": "UniProtKB:O00470"
}